4-hydroxyindole-3- carbonyl nitrile biosynthesis [GO:0106148] (biological process) Relationships: is a type of cyanogenic glycoside biosynthetic process [GO:0019756] References: PMID:26352477 Sources: GOC:lr Definition: The chemical reactions and pathways resulting in the formation of 4-hydroxyindole-3- carbonyl nitrile (4-OH-ICN), a cyanogenic glucoside.